seed trichome initiation [GO:0090377] (biological process) Definition: The process in which the developmental fate of an epidermal cell becomes restricted such that it will develop into a seed trichome, causing a change in the orientation of cell division in the ovule epidermis at or just before anthesis. Relationships: is a type of developmental process involved in reproduction [GO:0003006]; is a type of cellular process involved in reproduction in multicellular organism [GO:0022412]; is a type of GO:0045165; is part of GO:0090376 Note: These processes continue up to 3 days post-anthesis (DPA) in Gossypium spp. Also known as: seed trichome fate commitment References: PMID:17905721